{
  "gene_name": "Taste receptor type 2 member 46",
  "term_id": "GO:0033038",
  "gene": "UniProtKB:P59540",
  "term_label": "bitter taste receptor activity",
  "gene_symbol": "TAS2R46"
}